{
  "term_label": "axonogenesis",
  "term_id": "GO:0007409",
  "gene": "UniProtKB:P20336",
  "gene_symbol": "RAB3A",
  "gene_name": "Ras-related protein Rab-3A"
}